{
  "gene_name": "Putative C-type lectin-like domain family 1",
  "term_label": "Unknown molecular function",
  "gene_symbol": "CLECL1P",
  "term_id": "UNKNOWN:0001",
  "gene": "UniProtKB:Q8IZS7"
}